{
  "gene_symbol": "EMP2",
  "term_id": "GO:0005737",
  "gene": "UniProtKB:P54851",
  "gene_name": "Epithelial membrane protein 2",
  "term_label": "cytoplasm"
}